{
  "term_id": "UNKNOWN:0003",
  "gene": "UniProtKB:Q9BQ61",
  "gene_symbol": "TRIR",
  "term_label": "Unknown cellular component",
  "gene_name": "Telomerase RNA component interacting RNase"
}